cytoplasmic side of medial-Golgi cisterna membrane [GO:0160279] (cellular component) References: PMID:28777890, PMID:34597626, PMID:39658747 Also known as: cytoplasmic face of Golgi medial cisterna membrane, cytoplasmic leaflet of Golgi medial cisterna membrane Relationships: is a type of cytoplasmic side of membrane [GO:0098562]; is part of Golgi medial cisterna membrane [GO:1990675] Definition: The membrane leaflet of the medial-Golgi cisternae that faces the cytoplasm participates in interactions with cytosolic proteins involved in membrane trafficking, vesicle docking, and cargo sorting.